{
  "term_id": "GO:0046323",
  "gene": "UniProtKB:Q6PXP3",
  "gene_name": "Solute carrier family 2, facilitated glucose transporter member 7",
  "gene_symbol": "SLC2A7",
  "term_label": "D-glucose import"
}